positive regulation of embryonic skeletal joint development [GO:1902764] (biological process) References: PMID:16575901 Sources: GOC:TermGenie, GOC:mr, GO_REF:0000058 Relationships: is a type of positive regulation of developmental process [GO:0051094]; is a type of regulation of embryonic skeletal joint development [GO:1902762]; positively regulates GO:0072498 Definition: Any process that activates or increases the frequency, rate or extent of embryonic skeletal joint development. Also known as: up regulation of embryonic skeletal joint development, up-regulation of embryonic skeletal joint development, upregulation of embryonic skeletal joint development, activation of embryonic skeletal joint development